{
  "term_id": "GO:0045601",
  "gene": "UniProtKB:Q96LR9",
  "term_label": "regulation of endothelial cell differentiation",
  "gene_symbol": "APOLD1",
  "gene_name": "Apolipoprotein L domain-containing protein 1"
}